{
  "gene": "UniProtKB:Q9UHA7",
  "gene_name": "Interleukin-36 alpha",
  "term_label": "immune response",
  "term_id": "GO:0006955",
  "gene_symbol": "IL36A"
}